{
  "gene_symbol": "DEFB114",
  "gene_name": "Beta-defensin 114",
  "term_id": "GO:0042742",
  "gene": "UniProtKB:Q30KQ6",
  "term_label": "defense response to bacterium"
}